{
  "term_id": "GO:0015747",
  "gene_name": "Sodium-dependent phosphate transport protein 4",
  "gene_symbol": "SLC17A3",
  "term_label": "urate transport",
  "gene": "UniProtKB:O00476"
}